{
  "term_id": "GO:0071816",
  "gene_symbol": "EMC2",
  "gene": "UniProtKB:Q15006",
  "term_label": "tail-anchored membrane protein insertion into ER membrane",
  "gene_name": "ER membrane protein complex subunit 2"
}